{
  "term_id": "UNKNOWN:0001",
  "gene_symbol": "INTS5",
  "gene": "UniProtKB:Q6P9B9",
  "term_label": "Unknown molecular function",
  "gene_name": "Integrator complex subunit 5"
}